{
  "gene_symbol": "AK4P3",
  "gene": "UniProtKB:A0A8I5KW96",
  "gene_name": "Adenylate kinase 4, mitochondrial",
  "term_label": "nucleoside triphosphate biosynthetic process",
  "term_id": "GO:0009142"
}